{
  "gene": "UniProtKB:Q9NZN3",
  "term_label": "early endosome",
  "term_id": "GO:0005769",
  "gene_symbol": "EHD3",
  "gene_name": "EH domain-containing protein 3"
}